{
  "term_id": "GO:0005886",
  "term_label": "plasma membrane",
  "gene_name": "Tomoregulin-1",
  "gene": "UniProtKB:Q8IYR6",
  "gene_symbol": "TMEFF1"
}